{
  "gene": "UniProtKB:Q96QK1",
  "term_label": "intracellular protein transport",
  "gene_name": "Vacuolar protein sorting-associated protein 35",
  "term_id": "GO:0006886",
  "gene_symbol": "VPS35"
}